migracytosis [GO:0140495] (biological process) References: PMID:25342562 Relationships: is a type of export from cell [GO:0140352] Subtypes: mitocytosis [GO:0160040] Definition: A cell migration-dependent mechanism for releasing cellular contents.